selenocysteine-tRNA ligase activity [GO:0098619] (MF) Relationships: is a type of aminoacyl-tRNA ligase activity [GO:0004812] Definition: Catalysis of the reaction: tRNASec + L-Ser + ATP = Ser-tRNASec + AMP + diphosphate. References: PMID:8890909, PMID:9431993, PMID:9637248